{
  "gene": "UniProtKB:O00487",
  "term_label": "metal-dependent deubiquitinase activity",
  "term_id": "GO:0140492",
  "gene_symbol": "PSMD14",
  "gene_name": "26S proteasome non-ATPase regulatory subunit 14"
}